{
  "gene_name": "V-type proton ATPase subunit e 2",
  "gene_symbol": "ATP6V0E2",
  "gene": "UniProtKB:Q8NHE4",
  "term_id": "GO:0046961",
  "term_label": "proton-transporting ATPase activity, rotational mechanism"
}